microbody lumen [GO:0031907] (cellular component) Definition: The volume enclosed by the membranes of a microbody. Subtypes: peroxisomal matrix [GO:0005782] Relationships: is a type of GO:0070013; is part of GO:0042579 Sources: GOC:mah